{
  "term_id": "UNKNOWN:0003",
  "gene_symbol": "SCYL3",
  "term_label": "Unknown cellular component",
  "gene": "UniProtKB:Q8IZE3",
  "gene_name": "Protein-associating with the carboxyl-terminal domain of ezrin"
}